{
  "term_id": "GO:0005634",
  "gene_symbol": "ZNF454",
  "term_label": "nucleus",
  "gene_name": "Zinc finger protein 454",
  "gene": "UniProtKB:Q8N9F8"
}